{
  "gene_name": "Cyclin-dependent kinase 3",
  "term_id": "GO:0005634",
  "gene_symbol": "CDK3",
  "term_label": "nucleus",
  "gene": "UniProtKB:Q00526"
}